{
  "term_label": "growth hormone receptor binding",
  "gene_symbol": "JAK3",
  "gene": "UniProtKB:P52333",
  "gene_name": "Tyrosine-protein kinase JAK3",
  "term_id": "GO:0005131"
}